negative regulation of ryanodine-sensitive calcium-release channel activity [GO:0060315] (biological process) Sources: GOC:BHF, GOC:dph, GOC:tb Relationships: is a type of GO:0051280; is_a regulation of ryanodine-sensitive calcium-release channel activity [GO:0060314]; is a type of negative regulation of calcium ion transmembrane transporter activity [GO:1901020]; RO_0002212 ryanodine-sensitive calcium-release channel activity [GO:0005219] Definition: Any process that decreases the activity of a ryanodine-sensitive calcium-release channel. The ryanodine-sensitive calcium-release channel catalyzes the transmembrane transfer of a calcium ion by a channel that opens when a ryanodine class ligand has been bound by the channel complex or one of its constituent parts.